{
  "gene": "UniProtKB:Q8IVS8",
  "gene_symbol": "GLYCTK",
  "term_id": "UNKNOWN:0002",
  "term_label": "Unknown biological process",
  "gene_name": "Glycerate kinase"
}